{
  "term_label": "protein folding in endoplasmic reticulum",
  "term_id": "GO:0034975",
  "gene_symbol": "ERO1B",
  "gene": "UniProtKB:Q86YB8",
  "gene_name": "ERO1-like protein beta"
}